{
  "gene_symbol": "ATG2A",
  "term_label": "autophagy of mitochondrion",
  "gene": "UniProtKB:Q2TAZ0",
  "term_id": "GO:0000422",
  "gene_name": "Autophagy-related protein 2 homolog A"
}